{
  "term_label": "regulation of transcription by RNA polymerase II",
  "gene_symbol": "FOXD4L4",
  "gene": "UniProtKB:Q8WXT5",
  "gene_name": "Forkhead box protein D4-like 4",
  "term_id": "GO:0006357"
}